positive regulation of protein binding [GO:0032092] (BP) Sources: GOC:mah Definition: Any process that activates or increases the frequency, rate or extent of protein binding. Also known as: up regulation of protein binding, up-regulation of protein binding, upregulation of protein binding, activation of protein binding, stimulation of protein binding Subtypes: positive regulation of actin filament binding [GO:1904531] Relationships: is a type of regulation of protein binding [GO:0043393]; is a type of positive regulation of binding [GO:0051099]; positively regulates protein binding [GO:0005515]